{
  "term_label": "Unknown biological process",
  "gene": "UniProtKB:Q9UGK3",
  "term_id": "UNKNOWN:0002",
  "gene_symbol": "STAP2",
  "gene_name": "Signal-transducing adaptor protein 2"
}